{
  "gene_name": "Thioredoxin-like protein 4A",
  "term_id": "GO:0046540",
  "gene_symbol": "TXNL4A",
  "gene": "UniProtKB:P83876",
  "term_label": "U4/U6 x U5 tri-snRNP complex"
}